phenylpyruvate decarboxylase activity [GO:0050177] (molecular function) Also known as: phenylpyruvate carboxy-lyase (phenylacetaldehyde-forming), phenylpyruvate carboxy-lyase activity Relationships: is a type of carboxy-lyase activity [GO:0016831] Definition: Catalysis of the reaction: phenylpyruvate = phenylacetaldehyde + CO2. Sources: EC:4.1.1.43, MetaCyc:PHENYLPYRUVATE-DECARBOXYLASE-RXN